{
  "term_label": "keratinocyte differentiation",
  "term_id": "GO:0030216",
  "gene_name": "Protein-glutamine gamma-glutamyltransferase K",
  "gene": "UniProtKB:P22735",
  "gene_symbol": "TGM1"
}